14betaH-scalarane-17alpha-19-diol synthase activity [GO:0102646] (molecular function) Definition: Catalysis of the reaction: 14betaH-scalarane-17alpha-19-diol = all-trans-geranylfarnesol + H2O. Relationships: is a type of hydro-lyase activity [GO:0016836] References: PMID:24200803 Sources: GOC:pz